{
  "gene_symbol": "DCK",
  "gene_name": "Deoxycytidine kinase",
  "gene": "UniProtKB:P27707",
  "term_label": "Unknown biological process",
  "term_id": "UNKNOWN:0002"
}